limb granular cell differentiation [GO:0060891] (biological process) Definition: The process in which a relatively unspecialized cell acquires specialized features of a limb epidermal granular cell. Sources: GOC:dph, GOC:sdb_2009, GOC:tb Relationships: is a type of keratinocyte differentiation [GO:0030216]; is part of limb epidermis development [GO:0060887]